{
  "gene": "UniProtKB:O15105",
  "term_label": "anatomical structure morphogenesis",
  "gene_name": "Mothers against decapentaplegic homolog 7",
  "term_id": "GO:0009653",
  "gene_symbol": "SMAD7"
}